{
  "term_id": "GO:0043679",
  "term_label": "axon terminus",
  "gene": "UniProtKB:P16389",
  "gene_name": "Potassium voltage-gated channel subfamily A member 2",
  "gene_symbol": "KCNA2"
}